{
  "term_id": "UNKNOWN:0003",
  "gene_name": "Zinc finger protein 212",
  "gene_symbol": "ZNF212",
  "gene": "UniProtKB:Q9UDV6",
  "term_label": "Unknown cellular component"
}